L-isoleucine transmembrane transporter activity [GO:0015188] (molecular function) Also known as: L-isoleucine transporter activity, isoleucine/valine:sodium symporter activity, leucine/isoleucine/valine porter activity, leucine/valine/isoleucine permease activity Relationships: is a type of neutral L-amino acid transmembrane transporter activity [GO:0015175]; is a type of GO:0015179; is a type of GO:0015658 Sources: GOC:ai, GOC:mtg_transport, ISBN:0815340729 Definition: Enables the transfer of L-isoleucine from one side of a membrane to the other. L-isoleucine is (2R*,3R*)-2-amino-3-methylpentanoic acid.